{
  "gene_symbol": "PRODH2",
  "term_id": "GO:0004657",
  "term_label": "proline dehydrogenase activity",
  "gene": "UniProtKB:Q9UF12",
  "gene_name": "Hydroxyproline dehydrogenase"
}